protein secretion by the type VIII secretion system [GO:0098777] (biological process) Definition: Protein secretion through the outer membrane via the mechanism used for the secretion of curli subunits. Subtypes: curli subunit secretion coupled to curli assembly [GO:0098778] References: PMID:19299134, PMID:24080089 Relationships: is a type of protein transport across the cell outer membrane [GO:0098776] Also known as: T8SS Note: This term is defined so as to leave open the possibility that things other than curli subunits are secreted via same secretory system as that used by curli subunits.